{
  "gene": "UniProtKB:O75460",
  "term_label": "RNA endonuclease activity",
  "term_id": "GO:0004521",
  "gene_name": "Serine_threonine-protein kinase_endoribonuclease IRE1",
  "gene_symbol": "ERN1"
}